{
  "gene_name": "Epidermal growth factor receptor substrate 15",
  "gene": "UniProtKB:P42566",
  "term_id": "GO:0005886",
  "term_label": "plasma membrane",
  "gene_symbol": "EPS15"
}